transmembrane receptor protein tyrosine kinase activator activity [GO:0030297] (molecular function) Relationships: is a type of GO:0030296; is a type of signaling receptor activator activity [GO:0030546]; positively regulates GO:0004714 Sources: GOC:mah Definition: Binds to and increases the activity of a transmembrane receptor protein tyrosine kinase.